{
  "gene": "UniProtKB:Q96AP0",
  "term_label": "negative regulation of telomere maintenance via telomerase",
  "gene_name": "Adrenocortical dysplasia protein homolog",
  "gene_symbol": "ACD",
  "term_id": "GO:0032211"
}